{
  "term_label": "tRNA binding",
  "term_id": "GO:0000049",
  "gene_name": "Cytoplasmic tRNA 2-thiolation protein 1",
  "gene_symbol": "CTU1",
  "gene": "UniProtKB:Q7Z7A3"
}